{
  "gene_name": "Serine protease 53",
  "gene_symbol": "PRSS53",
  "term_id": "GO:0004252",
  "gene": "UniProtKB:Q2L4Q9",
  "term_label": "serine-type endopeptidase activity"
}